{
  "gene_symbol": "SLC5A10",
  "gene": "UniProtKB:A0PJK1",
  "gene_name": "Sodium_mannose cotransporter SLC5A10",
  "term_id": "GO:0140929",
  "term_label": "mannose:sodium symporter activity"
}